{
  "term_label": "Unknown cellular component",
  "gene": "UniProtKB:Q8NGD4",
  "term_id": "UNKNOWN:0003",
  "gene_name": "Olfactory receptor 4K1",
  "gene_symbol": "OR4K1"
}